{
  "gene_symbol": "A0A804HI29",
  "term_label": "Unknown biological process",
  "term_id": "UNKNOWN:0002",
  "gene_name": "Uncharacterized protein",
  "gene": "UniProtKB:A0A804HI29"
}